{
  "gene_symbol": "LAPTM4A",
  "gene": "UniProtKB:Q15012",
  "term_label": "regulation of lysosomal membrane permeability",
  "term_id": "GO:0097213",
  "gene_name": "Lysosomal-associated transmembrane protein 4A"
}